{
  "gene": "UniProtKB:Q6ZMI3",
  "gene_name": "Gliomedin",
  "term_id": "GO:0007165",
  "gene_symbol": "GLDN",
  "term_label": "signal transduction"
}